leaflet formation [GO:0090014] (biological process) Regulation: positively regulated by GO:0090015; regulated by regulation of leaflet formation [GO:0090016] Definition: The developmental process pertaining to the initial formation of a leaflet from unspecified parts. A leaflet is one of the ultimate segments of a compound leaf. Sources: GOC:dph, GOC:sdb_2009, GOC:tb Relationships: is a type of anatomical structure formation involved in morphogenesis [GO:0048646]; is part of leaflet morphogenesis [GO:0060794]